ADP-glucose pyrophosphohydrolase activity [GO:0080042] (molecular function) Definition: Catalysis of the reaction: ADP-glucose + H2O = AMP + glucose-1-phosphate. Relationships: is a type of ADP-sugar diphosphatase activity [GO:0019144] Sources: GOC:tb